{
  "term_id": "GO:0005634",
  "gene_name": "Kinesin-like protein KIF20A",
  "term_label": "nucleus",
  "gene_symbol": "KIF20A",
  "gene": "UniProtKB:O95235"
}